P2Y2 nucleotide receptor binding [GO:0031813] (molecular function) Definition: Binding to a P2Y2 nucleotide receptor. Also known as: P2Y2 nucleotide receptor ligand Relationships: is a type of G protein-coupled nucleotide receptor binding [GO:0031811] Sources: GOC:mah, GOC:nln